{
  "gene_symbol": "PSTPIP2",
  "term_label": "plasma membrane",
  "term_id": "GO:0005886",
  "gene": "UniProtKB:Q9H939",
  "gene_name": "Proline-serine-threonine phosphatase-interacting protein 2"
}